{
  "gene": "UniProtKB:O15375",
  "gene_name": "Monocarboxylate transporter 6",
  "term_id": "UNKNOWN:0002",
  "term_label": "Unknown biological process",
  "gene_symbol": "SLC16A5"
}